{
  "gene": "UniProtKB:O94777",
  "term_id": "GO:0180047",
  "term_label": "dolichol phosphate mannose biosynthetic process",
  "gene_name": "Dolichol phosphate-mannose biosynthesis regulatory protein",
  "gene_symbol": "DPM2"
}